{
  "term_label": "cytoplasm",
  "term_id": "GO:0005737",
  "gene": "UniProtKB:Q8WZ73",
  "gene_symbol": "RFFL",
  "gene_name": "E3 ubiquitin-protein ligase rififylin"
}